{
  "gene_symbol": "TFPI",
  "gene_name": "Tissue factor pathway inhibitor",
  "term_id": "GO:0004867",
  "gene": "UniProtKB:P10646",
  "term_label": "serine-type endopeptidase inhibitor activity"
}